{
  "gene_name": "Krueppel-like factor 17",
  "term_id": "GO:0005634",
  "gene": "UniProtKB:Q5JT82",
  "term_label": "nucleus",
  "gene_symbol": "KLF17"
}